{
  "gene": "UniProtKB:Q53TN4",
  "gene_name": "Plasma membrane ascorbate-dependent reductase CYBRD1",
  "term_id": "GO:0016491",
  "term_label": "oxidoreductase activity",
  "gene_symbol": "CYBRD1"
}